{
  "term_label": "neurogenesis",
  "gene_symbol": "FGF3",
  "gene_name": "Fibroblast growth factor 3",
  "term_id": "GO:0022008",
  "gene": "UniProtKB:P11487"
}